{
  "gene_name": "Ras-related protein Rab-6C",
  "gene_symbol": "RAB6C",
  "gene": "UniProtKB:Q9H0N0",
  "term_id": "GO:0006886",
  "term_label": "intracellular protein transport"
}